{
  "gene": "UniProtKB:Q9ULJ8",
  "term_label": "actin filament binding",
  "gene_symbol": "PPP1R9A",
  "term_id": "GO:0051015",
  "gene_name": "Neurabin-1"
}